{
  "gene_name": "Protein ENTREP3",
  "gene": "UniProtKB:P81408",
  "term_label": "Unknown biological process",
  "term_id": "UNKNOWN:0002",
  "gene_symbol": "ENTREP3"
}